{
  "gene_symbol": "ASB16",
  "term_id": "UNKNOWN:0001",
  "term_label": "Unknown molecular function",
  "gene": "UniProtKB:Q96NS5",
  "gene_name": "Ankyrin repeat and SOCS box protein 16"
}